{
  "gene": "UniProtKB:Q96N87",
  "gene_name": "Inactive sodium-dependent neutral amino acid transporter B(0)AT3",
  "term_id": "GO:0005886",
  "term_label": "plasma membrane",
  "gene_symbol": "SLC6A18"
}